{
  "term_id": "GO:0070301",
  "gene_symbol": "OSER1",
  "gene": "UniProtKB:Q9NX31",
  "term_label": "cellular response to hydrogen peroxide",
  "gene_name": "Oxidative stress-responsive serine-rich protein 1"
}